posterior lateral line neuromast primordium migration [GO:0048920] (biological process) Relationships: is a type of neuromast primordium migration [GO:0048883]; is part of posterior lateral line development [GO:0048916] Definition: The migration of a relatively undifferentiated cell along the developing posterior lateral line, originating from cranial ectodermal placodes situated behind the ear. The neuromast primordium deposits proneuromasts along the lateral line, from which the neuromasts will develop. References: PMID:15832385 Sources: GOC:dgh Also known as: PLL neuromast primordium migration